{
  "term_id": "GO:0005777",
  "gene": "UniProtKB:Q8N5R6",
  "gene_symbol": "CCDC33",
  "term_label": "peroxisome",
  "gene_name": "Coiled-coil domain-containing protein 33"
}